{
  "term_label": "cell differentiation",
  "gene_symbol": "CHRDL2",
  "term_id": "GO:0030154",
  "gene_name": "Chordin-like protein 2",
  "gene": "UniProtKB:Q6WN34"
}